{
  "term_label": "RNA polymerase II CTD heptapeptide repeat kinase activity",
  "term_id": "GO:0008353",
  "gene_symbol": "CDK7",
  "gene": "UniProtKB:P50613",
  "gene_name": "Cyclin-dependent kinase 7"
}